lateral shield [GO:0097569] (cellular component) Note: Note that we deem cilium and microtubule-based flagellum to be equivalent. Also note that, due to the asymmetric nature of the Giardia trophozoite, this term is defined spatially as the trophozoite is viewed from the dorsal side, with the two nuclei dorsal to the ventral disc, and the ventral disc toward the anterior. Relationships: is a type of cellular anatomical structure [GO:0110165]; is part of cell body [GO:0044297] Sources: GOC:giardia, ISBN:9780124260207 Definition: Region of the ventral side of the cell body found in Giardia species (trophozoite stage). It is located posterior on either side of the ventral groove; the upper boundary is the ventral disc, and the lower boundary is marked by the posteriolateral flagella.